2-hydroxybenzoyl-CoA biosynthetic process [GO:1901887] (biological process) Relationships: is a type of phenol-containing compound biosynthetic process [GO:0046189]; is a type of GO:0071616 Definition: The chemical reactions and pathways resulting in the formation of 2-hydroxybenzoyl-CoA. References: PMID:19757094 Sources: GOC:TermGenie Also known as: 2-hydroxybenzoyl-CoA anabolism, 2-hydroxybenzoyl-CoA biosynthesis, 2-hydroxybenzoyl-CoA formation, 2-hydroxybenzoyl-CoA synthesis